positive regulation of mitotic spindle pole body separation [GO:0010696] (biological process) Also known as: positive regulation of SPB separation References: PMID:16792804, PMID:18500339 Sources: GOC:dph, GOC:tb Relationships: is a type of GO:0010695; is a type of GO:0090068; positively regulates initial mitotic spindle pole body separation [GO:0000073] Definition: Any process that increases the rate, frequency or extent of the process involving the release of duplicated mitotic spindle pole bodies (SPBs) and their migration away from each other within the nuclear membrane.